{
  "term_id": "GO:0002161",
  "gene_name": "Alanine--tRNA ligase, cytoplasmic",
  "gene_symbol": "AARS1",
  "term_label": "aminoacyl-tRNA deacylase activity",
  "gene": "UniProtKB:P49588"
}